{
  "gene": "UniProtKB:Q9ULL1",
  "term_id": "UNKNOWN:0003",
  "gene_symbol": "PLEKHG1",
  "term_label": "Unknown cellular component",
  "gene_name": "Pleckstrin homology domain-containing family G member 1"
}